{
  "gene": "UniProtKB:Q9UIV8",
  "term_label": "Unknown molecular function",
  "term_id": "UNKNOWN:0001",
  "gene_symbol": "SERPINB13",
  "gene_name": "Serpin B13"
}